{
  "term_label": "peptide YY receptor activity",
  "gene_name": "Neuropeptide Y receptor type 4",
  "gene": "UniProtKB:P50391",
  "gene_symbol": "NPY4R",
  "term_id": "GO:0001601"
}